response to ximelagatran [GO:0036288] (biological process) Sources: GOC:hp Definition: Any process that results in a change in state or activity of a cell or an organism (in terms of movement, secretion, enzyme production, gene expression, etc.) as a result of a ximelagatran stimulus. Note: Note that this term is in the subset of terms that should not be used for direct manual annotation of gene products. It was created to be used for cross-referencing by other ontologies. Direct annotations to this term may be amended during annotation QC. Relationships: is a type of GO:1901698; is a type of response to oxygen-containing compound [GO:1901700]